{
  "term_id": "GO:0032868",
  "term_label": "response to insulin",
  "gene_name": "Solute carrier family 2, facilitated glucose transporter member 1",
  "gene_symbol": "SLC2A1",
  "gene": "UniProtKB:P11166"
}